{
  "term_label": "signal transduction",
  "gene": "UniProtKB:P14317",
  "gene_symbol": "HCLS1",
  "term_id": "GO:0007165",
  "gene_name": "Hematopoietic lineage cell-specific protein"
}